{
  "gene_name": "Espin",
  "gene_symbol": "ESPN",
  "gene": "UniProtKB:B1AK53",
  "term_label": "actin filament bundle assembly",
  "term_id": "GO:0051017"
}